{
  "term_id": "UNKNOWN:0003",
  "term_label": "Unknown cellular component",
  "gene_name": "Speedy protein E12",
  "gene": "UniProtKB:P0DUX1",
  "gene_symbol": "SPDYE12"
}